{
  "term_id": "GO:0005634",
  "gene": "UniProtKB:P16415",
  "gene_name": "Zinc finger protein 823",
  "gene_symbol": "ZNF823",
  "term_label": "nucleus"
}